peptidyl-arginine phosphorylation [GO:0018109] (BP) Definition: The phosphorylation of peptidyl-arginine to form omega-N-phospho-L-arginine. Sources: RESID:AA0222 Relationships: is a type of protein phosphorylation [GO:0006468]; is a type of GO:0018195